{
  "gene_name": "Vinculin",
  "gene_symbol": "VCL",
  "term_id": "GO:0005912",
  "gene": "UniProtKB:P18206",
  "term_label": "adherens junction"
}